{
  "gene_symbol": "SYCP2L",
  "gene_name": "Synaptonemal complex protein 2-like",
  "term_id": "UNKNOWN:0002",
  "gene": "UniProtKB:Q5T4T6",
  "term_label": "Unknown biological process"
}